{
  "gene_symbol": "HILPDA",
  "term_id": "GO:0035425",
  "gene_name": "Hypoxia-inducible lipid droplet-associated protein",
  "gene": "UniProtKB:Q9Y5L2",
  "term_label": "autocrine signaling"
}